{
  "gene_name": "Fibroblast growth factor 7",
  "gene": "UniProtKB:P21781",
  "term_id": "GO:0043410",
  "term_label": "positive regulation of MAPK cascade",
  "gene_symbol": "FGF7"
}